{
  "gene_symbol": "A0A8I5QKQ9",
  "term_label": "Unknown cellular component",
  "gene": "UniProtKB:A0A8I5QKQ9",
  "term_id": "UNKNOWN:0003",
  "gene_name": "Uncharacterized protein"
}